zinc ion import across plasma membrane [GO:0071578] (biological process) Regulation: regulated by regulation of zinc ion transmembrane import [GO:0071581]; negatively regulated by negative regulation of zinc ion transmembrane import [GO:0071584] Definition: The directed movement of zinc(2+) ions from outside of a cell, across the plasma membrane and into the cytosol. References: PMID:18637840 Sources: GOC:vw Relationships: is a type of zinc ion transmembrane transport [GO:0071577]; is a type of GO:0098659 Also known as: zinc II ion plasma membrane import, zinc II ion transmembrane import, zinc import, zinc ion import into cell, zinc uptake, high-affinity zinc II ion transmembrane import, high-affinity zinc II ion transport, low-affinity zinc II ion transport, zinc ion transmembrane import